{
  "gene_name": "Zinc finger protein 77",
  "term_id": "GO:0000977",
  "gene_symbol": "ZNF77",
  "gene": "UniProtKB:Q15935",
  "term_label": "RNA polymerase II transcription regulatory region sequence-specific DNA binding"
}